{
  "gene_symbol": "RNFT2",
  "gene": "UniProtKB:Q96EX2",
  "gene_name": "RING finger and transmembrane domain-containing protein 2",
  "term_label": "ubiquitin protein ligase activity",
  "term_id": "GO:0061630"
}